{
  "term_id": "GO:0010389",
  "gene": "UniProtKB:P49454",
  "term_label": "regulation of G2/M transition of mitotic cell cycle",
  "gene_symbol": "CENPF",
  "gene_name": "Centromere protein F"
}